{
  "term_id": "UNKNOWN:0002",
  "term_label": "Unknown biological process",
  "gene": "UniProtKB:Q6DCA0",
  "gene_name": "AMMECR1-like protein",
  "gene_symbol": "AMMECR1L"
}